D-glucarate transmembrane transporter activity [GO:0042878] (molecular function) Sources: GOC:jl, GOC:jsg, GOC:mah, GOC:mtg_transport, ISBN:0198506732 Definition: Enables the transfer of D-glucarate, the D-enantiomer of glucarate, from one side of a membrane to the other. Relationships: is a type of GO:0005310; is a type of carbohydrate transmembrane transporter activity [GO:0015144]; is a type of aldarate transmembrane transporter activity [GO:0042876]; BFO_0000050 D-glucarate transmembrane transport [GO:0042870]